synaptonemal complex organization [GO:0070193] (biological process) Relationships: is a type of chromosome organization [GO:0051276] Also known as: synaptonemal complex organisation Sources: GOC:mah Definition: A process that is carried out at the cellular level which results in the assembly, arrangement of constituent parts, or disassembly of a synaptonemal complex. A synaptonemal complex is a proteinaceous scaffold formed between homologous chromosomes during meiosis. Subtypes: synaptonemal complex assembly [GO:0007130], synaptonemal complex disassembly [GO:0070194]